{
  "term_label": "Unknown molecular function",
  "term_id": "UNKNOWN:0001",
  "gene_name": "Beta-defensin 131A",
  "gene": "UniProtKB:P59861",
  "gene_symbol": "DEFB131A"
}